{
  "term_label": "detection of chemical stimulus involved in sensory perception of smell",
  "gene_name": "Olfactory receptor 2G6",
  "gene_symbol": "OR2G6",
  "term_id": "GO:0050911",
  "gene": "UniProtKB:Q5TZ20"
}